{
  "term_label": "Unknown biological process",
  "gene_symbol": "GOLGB1",
  "gene_name": "Golgin subfamily B member 1",
  "term_id": "UNKNOWN:0002",
  "gene": "UniProtKB:Q14789"
}